ABC-type iron-sulfur cluster transporter activity [GO:0140481] (MF) Also known as: ATPase-coupled Fe-S cluster transmembrane transporter activity, ATPase-coupled iron-sulfur cluster transmembrane transporter activity References: PMID:31040179 Relationships: is a type of ABC-type transporter activity [GO:0140359] Definition: Catalysis of the reaction: ATP + H2O + iron-sulfur cluster(in) = ADP + phosphate + iron-sulfur cluster(out).